replication fork arrest at mating type locus [GO:0011000] (biological process) Definition: A process that impedes the progress of the DNA replication fork at natural replication fork pausing sites within the mating type locus. Relationships: is a type of replication fork arrest [GO:0043111] Sources: GOC:dph, GOC:tb